{
  "gene_name": "Leukocyte surface antigen CD47",
  "gene": "UniProtKB:Q08722",
  "term_label": "extracellular exosome",
  "gene_symbol": "CD47",
  "term_id": "GO:0070062"
}